{
  "term_id": "GO:0005783",
  "gene": "UniProtKB:Q9Y3E0",
  "gene_name": "Vesicle transport protein GOT1B",
  "term_label": "endoplasmic reticulum",
  "gene_symbol": "GOLT1B"
}